{
  "gene_symbol": "CARM1",
  "term_id": "UNKNOWN:0003",
  "gene_name": "Histone-arginine methyltransferase CARM1",
  "gene": "UniProtKB:Q86X55",
  "term_label": "Unknown cellular component"
}